peptidyl-cysteine acetylation [GO:0018533] (biological process) Sources: GOC:mah Relationships: is a type of protein acetylation [GO:0006473]; is a type of peptidyl-cysteine modification [GO:0018198] Definition: The acetylation of peptidyl-cysteine.